{
  "gene_symbol": "QDPR",
  "term_id": "GO:0070402",
  "gene": "UniProtKB:P09417",
  "gene_name": "Dihydropteridine reductase",
  "term_label": "NADPH binding"
}